adrenomedullin receptor binding [GO:0031700] (molecular function) Definition: Binding to an adrenomedullin receptor. Also known as: adrenomedullin receptor ligand Relationships: is a type of GO:0001664 Sources: GOC:mah, GOC:nln